spore wall assembly [GO:0042244] (biological process) Subtypes: ascospore wall assembly [GO:0030476], sexual spore wall assembly [GO:0034294], asexual spore wall assembly [GO:0042243] Relationships: is a type of cellular component assembly involved in morphogenesis [GO:0010927]; is a type of GO:0070726; is part of spore wall biogenesis [GO:0070590] Sources: GOC:mah, GOC:pg Definition: The aggregation, arrangement and bonding together of a set of components to form a spore wall; a spore wall is the specialized envelope lying outside the cell membrane of a spore. Also known as: spore coat biosynthesis, spore coat biosynthetic process, spore wall formation